positive regulation of peripheral B cell deletion [GO:0002910] (biological process) Relationships: is a type of GO:0002660; is a type of positive regulation of B cell mediated immunity [GO:0002714]; is a type of positive regulation of B cell deletion [GO:0002869]; is a type of regulation of peripheral B cell deletion [GO:0002908]; positively regulates GO:0002454 Also known as: up regulation of peripheral B cell deletion, up-regulation of peripheral B cell deletion, upregulation of peripheral B cell deletion, activation of peripheral B cell deletion, stimulation of peripheral B cell deletion Sources: GOC:add Definition: Any process that activates or increases the frequency, rate, or extent of peripheral B cell deletion.